{
  "gene_symbol": "SLC35F2",
  "gene": "UniProtKB:Q8IXU6",
  "term_id": "UNKNOWN:0001",
  "gene_name": "Solute carrier family 35 member F2",
  "term_label": "Unknown molecular function"
}